{
  "gene_name": "Proepiregulin",
  "gene_symbol": "EREG",
  "term_id": "GO:0007173",
  "gene": "UniProtKB:O14944",
  "term_label": "epidermal growth factor receptor signaling pathway"
}